nuclear receptor-mediated glucocorticoid signaling pathway [GO:0042921] (biological process) Relationships: is a type of nuclear receptor-mediated corticosteroid signaling pathway [GO:0031958] Also known as: glucocorticoid receptor signaling pathway, glucocorticoid receptor signalling pathway, intracellular glucocorticoid receptor signaling pathway Regulation: regulated by regulation of nuclear receptor-mediated glucocorticoid signaling pathway [GO:2000322]; negatively regulated by GO:2000323; positively regulated by GO:2000324 Definition: A nuclear receptor-mediated signaling pathway initiated by a glucocorticoid binding to an intracellular receptor of the nuclear receptor protein family, and ending with regulation of a downstream cellular process, e.g. transcription. References: PMID:15240347